epicardial cell to mesenchymal cell transition [GO:0003347] (biological process) References: PMID:18722343 Sources: GOC:dph Relationships: is a type of GO:0001837 Definition: A transition where an epicardial cell loses apical/basolateral polarity, severs intercellular adhesive junctions, degrades basement membrane components and becomes a migratory mesenchymal cell. The epicardium is a part of the pericardium.